{
  "term_label": "nuclear receptor activity",
  "term_id": "GO:0004879",
  "gene_name": "Nuclear receptor subfamily 1 group I member 3",
  "gene_symbol": "NR1I3",
  "gene": "UniProtKB:Q14994"
}